{
  "gene": "UniProtKB:Q5VU43",
  "term_label": "centrosome",
  "gene_symbol": "PDE4DIP",
  "gene_name": "Myomegalin",
  "term_id": "GO:0005813"
}